{
  "gene": "UniProtKB:O95235",
  "gene_symbol": "KIF20A",
  "gene_name": "Kinesin-like protein KIF20A",
  "term_id": "GO:0003777",
  "term_label": "microtubule motor activity"
}